{
  "term_label": "potassium ion homeostasis",
  "gene_symbol": "SLC12A2",
  "term_id": "GO:0055075",
  "gene": "UniProtKB:P55011",
  "gene_name": "Solute carrier family 12 member 2"
}